{
  "gene_symbol": "GTF3C5",
  "gene_name": "General transcription factor 3C polypeptide 5",
  "gene": "UniProtKB:Q9Y5Q8",
  "term_label": "transcription factor TFIIIC complex",
  "term_id": "GO:0000127"
}